positive regulation of cardiac endothelial to mesenchymal transition [GO:0062000] (biological process) Relationships: is a type of positive regulation of cell differentiation [GO:0045597]; is a type of positive regulation of multicellular organismal process [GO:0051240]; is_a regulation of cardiac endothelial to mesenchymal transition [GO:0061999]; positively regulates GO:0140074 References: PMID:26857067 Sources: GOC:BHF, GOC:BHF_miRNA, GOC:rph Definition: Any process that activates or increases the frequency, rate or extent of cardiac endothelial to mesenchymal trnasition.